{
  "gene": "UniProtKB:Q9UIF8",
  "gene_name": "Bromodomain adjacent to zinc finger domain protein 2B",
  "term_id": "UNKNOWN:0001",
  "gene_symbol": "BAZ2B",
  "term_label": "Unknown molecular function"
}